{
  "term_id": "GO:0005884",
  "gene_name": "Beta-actin-like protein 2",
  "gene": "UniProtKB:Q562R1",
  "gene_symbol": "ACTBL2",
  "term_label": "actin filament"
}